{
  "term_id": "GO:0003723",
  "gene_symbol": "CWC15",
  "gene": "UniProtKB:Q9P013",
  "term_label": "RNA binding",
  "gene_name": "Spliceosome-associated protein CWC15 homolog"
}